{
  "gene_symbol": "STRIP2",
  "gene_name": "Striatin-interacting protein 2",
  "term_id": "GO:0005829",
  "gene": "UniProtKB:Q9ULQ0",
  "term_label": "cytosol"
}